CD8 receptor binding [GO:0042610] (molecular function) Relationships: is a type of signaling receptor binding [GO:0005102] Definition: Binding to a CD8, a receptor found on the surface of thymocytes and cytotoxic and suppressor T-lymphocytes. Sources: GOC:jl, MSH:D016827